{
  "gene": "UniProtKB:P12236",
  "gene_name": "ADP_ATP translocase 3",
  "term_label": "ATP:ADP antiporter activity",
  "gene_symbol": "SLC25A6",
  "term_id": "GO:0005471"
}